tRNA pseudouridine synthesis [GO:0031119] (biological process) Relationships: is a type of GO:0001522; is a type of tRNA modification [GO:0006400] Sources: GOC:mah Subtypes: GO:0070902 Definition: The intramolecular conversion of uridine to pseudouridine in a tRNA molecule.